{
  "gene_symbol": "RIC1",
  "term_label": "retrograde transport, endosome to Golgi",
  "term_id": "GO:0042147",
  "gene": "UniProtKB:Q4ADV7",
  "gene_name": "Guanine nucleotide exchange factor subunit RIC1"
}